{
  "gene_name": "Actin-related protein 2",
  "term_label": "cell cortex",
  "term_id": "GO:0005938",
  "gene_symbol": "ACTR2",
  "gene": "UniProtKB:P61160"
}